{
  "gene": "UniProtKB:Q53ET0",
  "term_id": "GO:0005634",
  "gene_name": "CREB-regulated transcription coactivator 2",
  "term_label": "nucleus",
  "gene_symbol": "CRTC2"
}